cortical granule [GO:0060473] (CC) Also known as: cortical vesicle Sources: GOC:dph Definition: A secretory vesicle that is stored under the cell membrane of an egg. These vesicles fuse with the egg plasma membrane as part of egg activation and are part of the block to polyspermy. Relationships: is a type of secretory granule [GO:0030141]